{
  "gene_symbol": "POLE3",
  "term_id": "GO:0008623",
  "term_label": "CHRAC",
  "gene": "UniProtKB:Q9NRF9",
  "gene_name": "DNA polymerase epsilon subunit 3"
}